{
  "gene_name": "Eukaryotic translation initiation factor 4 gamma 2",
  "gene_symbol": "EIF4G2",
  "gene": "UniProtKB:P78344",
  "term_id": "GO:0006413",
  "term_label": "translational initiation"
}